{
  "term_label": "articular cartilage development",
  "gene_symbol": "OGN",
  "gene_name": "Mimecan",
  "gene": "UniProtKB:P20774",
  "term_id": "GO:0061975"
}